{
  "gene": "UniProtKB:P49959",
  "gene_name": "Double-strand break repair protein MRE11",
  "term_label": "meiotic DNA double-strand break formation",
  "gene_symbol": "MRE11",
  "term_id": "GO:0042138"
}